has ontology root term [IAO:0000700] (external)